{
  "term_id": "GO:0043565",
  "gene_symbol": "CHCHD2",
  "gene": "UniProtKB:Q9Y6H1",
  "gene_name": "Coiled-coil-helix-coiled-coil-helix domain-containing protein 2",
  "term_label": "sequence-specific DNA binding"
}